response to increased oxygen levels [GO:0036296] (biological process) Definition: Any process that results in a change in state or activity of a cell or an organism (in terms of movement, secretion, enzyme production, gene expression, etc.) as a result of a stimulus reflecting an increase in the level of oxygen. Sources: GOC:al Also known as: response to raised oxygen levels Note: This term should be used when an increase in oxygen levels is not considered a stress response. For a hyperoxic stress response, consider instead 'response to hyperoxia ; GO:0055093. Relationships: is a type of response to oxygen levels [GO:0070482] Subtypes: cellular response to increased oxygen levels [GO:0036295], response to hyperoxia [GO:0055093]